{
  "gene_name": "Zinc finger and BTB domain-containing protein 10",
  "gene_symbol": "ZBTB10",
  "gene": "UniProtKB:Q96DT7",
  "term_id": "GO:0000122",
  "term_label": "negative regulation of transcription by RNA polymerase II"
}